{
  "gene": "UniProtKB:Q9Y235",
  "term_label": "cytidine to uridine editing",
  "term_id": "GO:0016554",
  "gene_name": "C-U-editing enzyme APOBEC-2",
  "gene_symbol": "APOBEC2"
}